{
  "gene_name": "Protocadherin alpha-11",
  "term_id": "GO:0007155",
  "gene": "UniProtKB:Q9Y5I1",
  "term_label": "cell adhesion",
  "gene_symbol": "PCDHA11"
}